{
  "term_label": "DNA binding",
  "term_id": "GO:0003677",
  "gene": "UniProtKB:Q8WXF8",
  "gene_symbol": "DEDD2",
  "gene_name": "DNA-binding death effector domain-containing protein 2"
}